{
  "gene_name": "NADPH oxidase 4",
  "term_id": "GO:0016175",
  "gene": "UniProtKB:Q9NPH5",
  "gene_symbol": "NOX4",
  "term_label": "superoxide-generating NAD(P)H oxidase activity"
}